{
  "gene_symbol": "FCER1A",
  "term_id": "GO:0016064",
  "term_label": "immunoglobulin mediated immune response",
  "gene_name": "High affinity immunoglobulin epsilon receptor subunit alpha",
  "gene": "UniProtKB:P12319"
}